{
  "term_label": "morphogenesis of an epithelium",
  "gene_name": "Keratin, type I cytoskeletal 25",
  "gene": "UniProtKB:Q7Z3Z0",
  "gene_symbol": "KRT25",
  "term_id": "GO:0002009"
}